radial spoke head 3 [GO:0120338] (cellular component) Definition: The portion of the radial spoke 3 that is orthogonal to the elongated stalk and which projects towards the central pair of microtubules within the ciliary axoneme. Relationships: is a type of radial spoke head [GO:0001535]; is part of radial spoke 3 [GO:0120335] Also known as: radial spokehead 3 References: PMID:22754630, PMID:348711799 Sources: GOC:krc